{
  "gene_name": "ATP-dependent translocase ABCB1",
  "term_label": "ceramide translocation",
  "gene_symbol": "ABCB1",
  "gene": "UniProtKB:P08183",
  "term_id": "GO:0099040"
}